early endosome to late endosome transport [GO:0045022] (biological process) References: PMID:29980602 Sources: ISBN:0815316194 Regulation: regulated by regulation of early endosome to late endosome transport [GO:2000641]; negatively regulated by negative regulation of early endosome to late endosome transport [GO:2000642]; positively regulated by positive regulation of early endosome to late endosome transport [GO:2000643] Also known as: endosome maturation Definition: The directed movement of substances, in membrane-bounded vesicles, from the early sorting endosomes to the late sorting endosomes; transport occurs along microtubules and can be experimentally blocked with microtubule-depolymerizing drugs. Relationships: is a type of vesicle-mediated transport between endosomal compartments [GO:0098927]; occurs in cytoplasm [GO:0005737]